{
  "term_id": "GO:0006357",
  "gene_name": "Mediator of RNA polymerase II transcription subunit 6",
  "term_label": "regulation of transcription by RNA polymerase II",
  "gene": "UniProtKB:O75586",
  "gene_symbol": "MED6"
}